{
  "gene_name": "Ribonuclease 3",
  "gene_symbol": "DROSHA",
  "term_id": "GO:0031054",
  "gene": "UniProtKB:Q9NRR4",
  "term_label": "pre-miRNA processing"
}